{
  "gene_name": "N-acetylglucosamine-1-phosphotransferase subunit gamma",
  "gene_symbol": "GNPTG",
  "term_label": "Unknown molecular function",
  "term_id": "UNKNOWN:0001",
  "gene": "UniProtKB:Q9UJJ9"
}